{
  "gene_symbol": "MEF2A",
  "gene_name": "Myocyte-specific enhancer factor 2A",
  "term_label": "cell differentiation",
  "gene": "UniProtKB:Q02078",
  "term_id": "GO:0030154"
}